{
  "term_id": "GO:0035591",
  "gene": "UniProtKB:P46109",
  "gene_symbol": "CRKL",
  "term_label": "signaling adaptor activity",
  "gene_name": "Crk-like protein"
}